{
  "gene_name": "Uncharacterized protein KIAA0232",
  "gene": "UniProtKB:Q92628",
  "term_label": "Unknown biological process",
  "gene_symbol": "KIAA0232",
  "term_id": "UNKNOWN:0002"
}